{
  "gene": "UniProtKB:P36941",
  "term_id": "GO:0031625",
  "gene_symbol": "LTBR",
  "term_label": "ubiquitin protein ligase binding",
  "gene_name": "Tumor necrosis factor receptor superfamily member 3"
}